beta-amyrin 11-oxidase activity [GO:0102289] (molecular function) Definition: Catalysis of the reaction: beta-amyrin + 2 O2 + 2 NADPH + 2 H+ = 11-oxo-beta-amyrin + 3 H2O + 2 NADP. Relationships: is a type of oxidoreductase activity, acting on paired donors, with incorporation or reduction of molecular oxygen, NAD(P)H as one donor, and incorporation of one atom of oxygen [GO:0016709] Sources: RHEA:31711